{
  "gene_symbol": "AQP6",
  "term_id": "UNKNOWN:0002",
  "gene": "UniProtKB:Q13520",
  "term_label": "Unknown biological process",
  "gene_name": "Aquaporin-6"
}